{
  "term_id": "GO:0045165",
  "gene": "UniProtKB:P35712",
  "gene_symbol": "SOX6",
  "term_label": "cell fate commitment",
  "gene_name": "Transcription factor SOX-6"
}